{
  "gene_symbol": "FOXD4L4",
  "gene_name": "Forkhead box protein D4-like 4",
  "term_label": "anatomical structure morphogenesis",
  "term_id": "GO:0009653",
  "gene": "UniProtKB:Q8WXT5"
}